chloroplast relocation [GO:0009902] (biological process) Also known as: chloroplast movement References: PMID:11309623 Definition: The process in which chloroplasts in photosynthetic cells migrate toward illuminated sites to optimize photosynthesis and move away from excessively illuminated areas to protect the photosynthetic machinery. Subtypes: chloroplast avoidance movement [GO:0009903], GO:0009904 Relationships: is a type of chloroplast organization [GO:0009658]; is a type of GO:0019750; is a type of establishment of plastid localization [GO:0051667]